host-mediated perturbation of viral genome replication [GO:0044827] (biological process) Sources: GOC:jl Definition: A process in which a host organism alters or subverts viral genome replication. Subtypes: host-mediated activation of viral genome replication [GO:0044829] Relationships: is a type of GO:0044788 Also known as: modulation by host of viral genome replication, regulation by host of viral genome reproduction